motor neuron migration [GO:0097475] (biological process) Definition: The orderly movement of a motor neuron from one site to another. A motor neuron is an efferent neuron that passes from the central nervous system or a ganglion toward or to a muscle and conducts an impulse that causes movement. Subtypes: spinal cord motor neuron migration [GO:0097476] Relationships: is a type of GO:0001764 References: PMID:20711475 Sources: CL:0000100, GOC:yaf Regulation: RO_0002211 by GO:1905483; negatively regulated by GO:1905484; positively regulated by positive regulation of motor neuron migration [GO:1905485]